{
  "term_label": "Unknown cellular component",
  "term_id": "UNKNOWN:0003",
  "gene_name": "Putative deoxyribonuclease TATDN2",
  "gene_symbol": "TATDN2",
  "gene": "UniProtKB:Q93075"
}